posterior lateral line nerve glial cell development [GO:0048941] (biological process) Definition: The process aimed at the progression of a glial cell in the posterior lateral line nerve over time, from initial commitment of the cell to a specific fate, to the fully functional differentiated cell. Sources: GOC:dgh Relationships: is a type of lateral line nerve glial cell development [GO:0048937]; is part of posterior lateral line nerve glial cell differentiation [GO:0048931]